{
  "gene_name": "Transcription factor Gibbin",
  "gene": "UniProtKB:Q5TGY3",
  "term_label": "Unknown biological process",
  "term_id": "UNKNOWN:0002",
  "gene_symbol": "AHDC1"
}